dopaminechrome tautomerase activity [GO:0106417] (molecular function) Definition: Catalysis of the reaction: dopaminechrome = 5,6-dihydroxyindole. References: PMID:34388859 Sources: RHEA:70199 Relationships: is a type of intramolecular oxidoreductase activity, transposing C=C bonds [GO:0016863]